{
  "term_label": "U1 snRNA 3'-end processing",
  "gene_name": "Exosome complex component RRP45",
  "gene": "UniProtKB:Q06265",
  "gene_symbol": "EXOSC9",
  "term_id": "GO:0034473"
}